sulfite reductase activity [GO:0016002] (molecular function) Definition: Catalysis of the reaction: hydrogen sulfide + acceptor + 3 H2O = sulfite + reduced acceptor. Relationships: is a type of oxidoreductase activity, acting on a sulfur group of donors [GO:0016667] Also known as: assimilatory sulfite reductase activity, assimilatory-type sulfite reductase activity, hydrogen-sulfide:(acceptor) oxidoreductase activity, hydrogen-sulfide:acceptor oxidoreductase activity, sulphite reductase activity Sources: GOC:curators Subtypes: sulfite reductase (NADPH) activity [GO:0004783]